{
  "gene": "UniProtKB:Q5MJ08",
  "term_label": "Unknown cellular component",
  "gene_symbol": "SPANXN4",
  "gene_name": "Sperm protein associated with the nucleus on the X chromosome N4",
  "term_id": "UNKNOWN:0003"
}